negative regulation of lymphocyte chemotaxis [GO:1901624] (biological process) Sources: GOC:TermGenie Also known as: down regulation of lymphocyte chemotaxis, down-regulation of lymphocyte chemotaxis, downregulation of lymphocyte chemotaxis, inhibition of lymphocyte chemotaxis Definition: Any process that stops, prevents or reduces the frequency, rate or extent of lymphocyte chemotaxis. Relationships: is a type of GO:0002689; is a type of regulation of lymphocyte chemotaxis [GO:1901623]; is a type of negative regulation of lymphocyte migration [GO:2000402]; negatively regulates lymphocyte chemotaxis [GO:0048247] Subtypes: negative regulation of natural killer cell chemotaxis [GO:2000502], negative regulation of B cell chemotaxis [GO:2000550]